adventitious septum [GO:0000933] (cellular component) Relationships: is_a cell septum [GO:0030428] Sources: GOC:clt, ISBN:0471940526 Definition: A cell septum whose formation is independent of nuclear division.